{
  "term_id": "GO:0005615",
  "gene": "UniProtKB:Q7Z5L7",
  "term_label": "extracellular space",
  "gene_symbol": "PODN",
  "gene_name": "Podocan"
}